{
  "gene": "UniProtKB:Q12923",
  "gene_symbol": "PTPN13",
  "gene_name": "Tyrosine-protein phosphatase non-receptor type 13",
  "term_label": "regulation of phosphatidylinositol 3-kinase/protein kinase B signal transduction",
  "term_id": "GO:0051896"
}